{
  "term_id": "GO:0004674",
  "gene": "UniProtKB:Q9H2X6",
  "gene_name": "Homeodomain-interacting protein kinase 2",
  "term_label": "protein serine/threonine kinase activity",
  "gene_symbol": "HIPK2"
}